{
  "term_label": "single fertilization",
  "gene_symbol": "TRPC7",
  "gene_name": "Short transient receptor potential channel 7",
  "term_id": "GO:0007338",
  "gene": "UniProtKB:Q9HCX4"
}